{
  "term_id": "GO:0007186",
  "gene_name": "Hydroxycarboxylic acid receptor 2",
  "gene_symbol": "HCAR2",
  "gene": "UniProtKB:Q8TDS4",
  "term_label": "G protein-coupled receptor signaling pathway"
}